{
  "term_id": "GO:0019814",
  "gene_symbol": "IGKV3D-7",
  "gene": "UniProtKB:A0A0C4DH55",
  "term_label": "immunoglobulin complex",
  "gene_name": "Immunoglobulin kappa variable 3D-7"
}